{
  "term_label": "Unknown molecular function",
  "term_id": "UNKNOWN:0001",
  "gene_name": "Cardiac-enriched FHL2-interacting protein",
  "gene": "UniProtKB:Q711Q0",
  "gene_symbol": "CEFIP"
}